central B cell negative selection [GO:0002354] (biological process) Also known as: central B lymphocyte negative selection, central B-cell negative selection, central B-lymphocyte negative selection Sources: GOC:jal Definition: Any process leading to negative selection of B cells in the bone marrow. Relationships: is a type of central B cell selection [GO:0002340]; is a type of B cell negative selection [GO:0002352]